{
  "gene": "UniProtKB:P28324",
  "gene_name": "ETS domain-containing protein Elk-4",
  "term_id": "GO:0000981",
  "gene_symbol": "ELK4",
  "term_label": "DNA-binding transcription factor activity, RNA polymerase II-specific"
}